positive regulation of mitochondrial translational elongation [GO:1905084] (biological process) Definition: Any process that activates or increases the frequency, rate or extent of mitochondrial translational elongation. Also known as: positive regulation of mitochondrial translation elongation, up regulation of mitochondrial translation elongation, up regulation of mitochondrial translational elongation, up-regulation of mitochondrial translation elongation, up-regulation of mitochondrial translational elongation, upregulation of mitochondrial translation elongation, upregulation of mitochondrial translational elongation, activation of mitochondrial translation elongation, activation of mitochondrial translational elongation References: PMID:25738458 Sources: GOC:TermGenie, GO_REF:0000058 Relationships: is a type of positive regulation of translational elongation [GO:0045901]; is a type of GO:1905082; positively regulates mitochondrial translational elongation [GO:0070125]